DNA strand exchange activity [GO:0000150] (molecular function) Definition: Catalysis of the identification and base-pairing of homologous sequences between single-stranded DNA and double-stranded DNA. Note: Note that this term represents activities that do not break or form phosphodiester bonds, and is therefore not a parent of 'site-specific recombinase activity ; GO:0009009'. Relationships: is a type of catalytic activity, acting on DNA [GO:0140097]; is part of DNA recombination [GO:0006310] Also known as: recombinase activity, strand transferase, RecA-family recombinase activity, strand exchange activity Regulation: positively regulated by DNA strand exchange activator activity [GO:0140619]; negatively regulated by GO:0140620 Sources: GOC:elh